{
  "term_label": "regulation of cytokine production",
  "gene_symbol": "BTN3A1",
  "gene": "UniProtKB:O00481",
  "gene_name": "Butyrophilin subfamily 3 member A1",
  "term_id": "GO:0001817"
}